{
  "term_id": "GO:0005741",
  "gene": "UniProtKB:Q14693",
  "gene_symbol": "LPIN1",
  "term_label": "mitochondrial outer membrane",
  "gene_name": "Phosphatidate phosphatase LPIN1"
}